{
  "gene_symbol": "ANKRD20A5P",
  "gene": "UniProtKB:A0PJZ0",
  "gene_name": "Putative ankyrin repeat domain-containing protein 20A5",
  "term_id": "UNKNOWN:0002",
  "term_label": "Unknown biological process"
}